{
  "gene": "UniProtKB:Q00005",
  "term_id": "UNKNOWN:0002",
  "term_label": "Unknown biological process",
  "gene_symbol": "PPP2R2B",
  "gene_name": "Serine_threonine-protein phosphatase 2A 55 kDa regulatory subunit B beta isoform"
}